{
  "term_label": "plasma membrane",
  "gene": "UniProtKB:P16066",
  "gene_symbol": "NPR1",
  "term_id": "GO:0005886",
  "gene_name": "Atrial natriuretic peptide receptor 1"
}